{
  "gene": "UniProtKB:Q9H492",
  "term_id": "GO:0000045",
  "gene_name": "Microtubule-associated proteins 1A_1B light chain 3A",
  "gene_symbol": "MAP1LC3A",
  "term_label": "autophagosome assembly"
}